metallochaperone activity [GO:0016530] (molecular function) Relationships: is_a GO:0140104; has part metal ion binding [GO:0046872] References: PMID:11739376 Subtypes: copper chaperone activity [GO:0016531], iron chaperone activity [GO:0034986], iron-sulfur cluster chaperone activity [GO:0140132], ATP-dependent FeS chaperone activity [GO:0140663], zinc chaperone activity [GO:0140827], nickel chaperone activity [GO:0170061] Definition: Binding to and delivering metal ions to a target protein.